inhibition of histamine uptake [GO:0051619] (biological process) Sources: GOC:ai Also known as: inhibition of histamine import Relationships: is a type of inhibition of neurotransmitter uptake [GO:0051609]; is a type of negative regulation of histamine uptake [GO:0051617] Definition: Any process that prevents the activation of the directed movement of histamine into a cell.